{
  "term_label": "Unknown cellular component",
  "gene": "UniProtKB:P0DV79",
  "gene_name": "Speedy protein E18",
  "term_id": "UNKNOWN:0003",
  "gene_symbol": "SPDYE18"
}